glucuronoxylan glucuronosyltransferase activity [GO:0080116] (molecular function) Definition: Catalysis of the transfer of glucuronate to the xylan backbone of glucuronoxylan molecule. Relationships: is_a glucuronosyltransferase activity [GO:0015020] References: PMID:18980649